eisosome assembly [GO:0070941] (biological process) Definition: The aggregation, arrangement and bonding together of a set of components to form an eisosome, a cell part that is composed of the eisosome membrane and eisosome filaments. The eisosome membrane, also called the MCC domain, is a furrow-like plasma membrane sub-domain with associated integral transmembrane proteins. The eisosome filaments form a scaffolding lattice on the cytoplasmic face of the membrane. References: PMID:19564405 Sources: GOC:al, GOC:jp, GOC:mah Relationships: is a type of GO:0022607